creatine transmembrane transport [GO:0015881] (biological process) Definition: The directed movement of creatine across a membrane. Sources: GOC:TermGenie, GOC:pr, GO_REF:0000069 Also known as: creatine transport Relationships: is a type of monocarboxylic acid transport [GO:0015718]; is_a modified amino acid transport [GO:0072337]; is a type of carboxylic acid transmembrane transport [GO:1905039]